{
  "gene": "UniProtKB:Q9H9J4",
  "gene_name": "Ubiquitin carboxyl-terminal hydrolase 42",
  "term_label": "regulation of protein stability",
  "term_id": "GO:0031647",
  "gene_symbol": "USP42"
}